{
  "gene_name": "DnaJ homolog subfamily A member 1",
  "term_id": "GO:0051087",
  "gene": "UniProtKB:P31689",
  "gene_symbol": "DNAJA1",
  "term_label": "protein-folding chaperone binding"
}